{
  "gene": "UniProtKB:P30968",
  "gene_name": "Gonadotropin-releasing hormone receptor",
  "term_label": "cellular response to hormone stimulus",
  "gene_symbol": "GNRHR",
  "term_id": "GO:0032870"
}